{
  "term_label": "Unknown molecular function",
  "term_id": "UNKNOWN:0001",
  "gene_name": "Usherin",
  "gene_symbol": "USH2A",
  "gene": "UniProtKB:O75445"
}